{
  "term_label": "cytoplasm",
  "gene_name": "Peroxiredoxin-like 2A",
  "gene": "UniProtKB:Q9BRX8",
  "term_id": "GO:0005737",
  "gene_symbol": "PRXL2A"
}